{
  "term_id": "GO:0007043",
  "gene": "UniProtKB:P55287",
  "gene_name": "Cadherin-11",
  "term_label": "cell-cell junction assembly",
  "gene_symbol": "CDH11"
}